{
  "term_label": "cytoplasm",
  "gene_name": "Peptidyl-prolyl cis-trans isomerase A-like 4D",
  "term_id": "GO:0005737",
  "gene_symbol": "PPIAL4D",
  "gene": "UniProtKB:F5H284"
}